positive regulation of myotome development [GO:2000287] (biological process) Definition: Any process that activates or increases the frequency, rate or extent of myotome development. Sources: GOC:BHF Relationships: is_a positive regulation of developmental process [GO:0051094]; is a type of regulation of myotome development [GO:2000290]; positively regulates myotome development [GO:0061055]